{
  "term_id": "GO:0045786",
  "gene_symbol": "GMNN",
  "term_label": "negative regulation of cell cycle",
  "gene_name": "Geminin",
  "gene": "UniProtKB:O75496"
}